{
  "term_id": "GO:0016197",
  "gene_symbol": "EPS15L1",
  "term_label": "endosomal transport",
  "gene": "UniProtKB:Q9UBC2",
  "gene_name": "Epidermal growth factor receptor substrate 15-like 1"
}